symbiont-mediated disruption of host cell nucleus [GO:0044066] (biological process) Definition: The process in which an organism effects a change that impairs the structure or function of the host cell nucleus. Sources: MITRE:tk Also known as: disruption by symbiont of host cell nucleus, modification by symbiont of host nucleus, modification of host cell nucleus by symbiont, modification of host nucleus by symbiont, modification by symbiont of host cell nucleus Relationships: is a type of symbiont-mediated disruption of host cellular anatomical structure [GO:0052008]